vacuolar proton-transporting V-type ATPase complex assembly [GO:0070072] (biological process) Definition: The aggregation, arrangement and bonding together of a vacuolar proton-transporting V-type ATPase complex, proton-transporting two-sector ATPase complex that couples ATP hydrolysis to the transport of protons across the vacuolar membrane. Relationships: is a type of proton-transporting V-type ATPase complex assembly [GO:0070070] Sources: GOC:BHF, GOC:mah Also known as: V-ATPase assembly, V-ATPase complex assembly